mineralocorticoid catabolic process [GO:0006712] (BP) Sources: ISBN:0198506732 Subtypes: aldosterone catabolic process [GO:0032343] Also known as: mineralocorticoid breakdown, mineralocorticoid catabolism, mineralocorticoid degradation Relationships: is a type of GO:0006706; is a type of mineralocorticoid metabolic process [GO:0008212]; is a type of hormone catabolic process [GO:0042447] Definition: The chemical reactions and pathways resulting in the breakdown of mineralocorticoids, hormonal C21 corticosteroids synthesized from cholesterol.